{
  "gene_symbol": "OPRL1",
  "gene": "UniProtKB:P41146",
  "term_id": "GO:0005886",
  "gene_name": "Nociceptin receptor",
  "term_label": "plasma membrane"
}